{
  "gene": "UniProtKB:Q53EP0",
  "gene_name": "Fibronectin type III domain-containing protein 3B",
  "term_id": "UNKNOWN:0001",
  "term_label": "Unknown molecular function",
  "gene_symbol": "FNDC3B"
}